{
  "gene": "UniProtKB:Q9NRD9",
  "term_id": "GO:0042554",
  "gene_symbol": "DUOX1",
  "gene_name": "Dual oxidase 1",
  "term_label": "superoxide anion generation"
}